{
  "term_label": "regulation of double-strand break repair via homologous recombination",
  "gene": "UniProtKB:Q86V20",
  "gene_name": "Shieldin complex subunit 2",
  "gene_symbol": "SHLD2",
  "term_id": "GO:0010569"
}